parathyroid hormone receptor binding [GO:0031856] (molecular function) Subtypes: type 1 parathyroid hormone receptor binding [GO:0031857] Definition: Binding to a parathyroid hormone receptor. Sources: GOC:mah, GOC:nln Relationships: is_a G protein-coupled receptor binding [GO:0001664] Also known as: parathyroid hormone receptor ligand